{
  "gene_symbol": "SEMA4C",
  "gene_name": "Semaphorin-4C",
  "term_id": "GO:0038191",
  "term_label": "neuropilin binding",
  "gene": "UniProtKB:Q9C0C4"
}